centriole [GO:0005814] (cellular component) Definition: A cellular organelle, found close to the nucleus in many eukaryotic cells, consisting of a small cylinder with microtubular walls, 300-500 nm long and 150-250 nm in diameter. It contains nine short, parallel, peripheral microtubular fibrils, each fibril consisting of one complete microtubule fused to two incomplete microtubules. Cells usually have two centrioles, lying at right angles to each other. At division, each pair of centrioles generates another pair and the twin pairs form the pole of the mitotic spindle. Sources: ISBN:0198547684 Note: In most eukaryotic cells, 'ciliary basal body' (GO:0036064) and 'centriole' (GO:0005814) represent a common entity that cycles through its function in cell division, then ciliogenesis, then cell division again. However, these structures are modified extensively as they transition into each other, and may contain different proteins, specific to each component. Relationships: is a type of intracellular membraneless organelle [GO:0043232]; is part of microtubule organizing center [GO:0005815] Also known as: daughter centriole, mother centriole